{
  "gene_name": "Tubulin-specific chaperone E",
  "gene": "UniProtKB:Q15813",
  "term_label": "tubulin complex assembly",
  "gene_symbol": "TBCE",
  "term_id": "GO:0007021"
}